negative regulation of apoptotic cell clearance [GO:2000426] (BP) Definition: Any process that stops, prevents or reduces the frequency, rate or extent of apoptotic cell clearance. Sources: GOC:obol Subtypes: negative regulation of engulfment of apoptotic cell [GO:1901075] Also known as: negative regulation of apoptotic cell removal, negative regulation of efferocytosis, negative regulation of programmed cell clearance Relationships: is a type of GO:0050765; is a type of regulation of apoptotic cell clearance [GO:2000425]; negatively regulates apoptotic cell clearance [GO:0043277]